{
  "gene_symbol": "TMEM74",
  "term_id": "UNKNOWN:0002",
  "gene": "UniProtKB:Q96NL1",
  "term_label": "Unknown biological process",
  "gene_name": "Transmembrane protein 74"
}